very-low-density lipoprotein particle [GO:0034361] (cellular component) Relationships: is a type of triglyceride-rich plasma lipoprotein particle [GO:0034385] Definition: A triglyceride-rich lipoprotein particle that is typically composed of APOB100, APOE and APOCs and has a density of about 1.006 g/ml and a diameter of between 20-80 nm. It is found in blood and transports endogenous products (newly synthesized cholesterol and triglycerides) from the liver. Also known as: VLDL complex, VLDL particle, very-low-density lipoprotein complex Sources: GOC:BHF, GOC:expert_pt, GOC:mah, GOC:rl